{
  "gene": "UniProtKB:Q63HM2",
  "term_id": "UNKNOWN:0001",
  "gene_symbol": "PCNX4",
  "term_label": "Unknown molecular function",
  "gene_name": "Pecanex-like protein 4"
}